{
  "term_id": "GO:0050839",
  "gene": "UniProtKB:P35241",
  "term_label": "cell adhesion molecule binding",
  "gene_name": "Radixin",
  "gene_symbol": "RDX"
}